{
  "gene": "UniProtKB:P63162",
  "term_label": "U4/U6 x U5 tri-snRNP complex",
  "term_id": "GO:0046540",
  "gene_symbol": "SNRPN",
  "gene_name": "Small nuclear ribonucleoprotein-associated protein N"
}